{
  "term_id": "UNKNOWN:0003",
  "gene_symbol": "KRTAP10-4",
  "term_label": "Unknown cellular component",
  "gene_name": "Keratin-associated protein 10-4",
  "gene": "UniProtKB:P60372"
}